{
  "gene_name": "24-hydroxycholesterol 7-alpha-hydroxylase",
  "gene_symbol": "CYP39A1",
  "term_id": "GO:0008395",
  "gene": "UniProtKB:Q9NYL5",
  "term_label": "steroid hydroxylase activity"
}